establishment of bipolar cell polarity involved in cell morphogenesis [GO:0061159] (biological process) Sources: GOC:dph, GOC:vw Definition: The specification and formation of bipolar intracellular organization or cell growth patterns that contribute to cell morphogenesis. Bipolar organization is the organization that is a mirror image along an axis from a plane. Relationships: is a type of establishment of bipolar cell polarity [GO:0061171]; is part of cell morphogenesis [GO:0000902]